{
  "term_id": "GO:0030627",
  "gene_name": "Pre-mRNA-processing factor 39",
  "term_label": "pre-mRNA 5'-splice site binding",
  "gene": "UniProtKB:Q86UA1",
  "gene_symbol": "PRPF39"
}